trans-o-hydroxybenzylidenepyruvate hydratase-aldolase activity [GO:0018813] (molecular function) Definition: Catalysis of the reaction: 2-oxo-3-enoate-4-benzenoid + H2O = pyruvate + benzaldehyde derivative. Substrates are (3E)-4-(5-amino-2-hydroxy-phenyl)-2-oxo-but-3-ene-1-oic-acid (forms 5-aminosalicylaldehyde) and trans-o-hydroxybenzylidenepyruvate (forms salicylaldehyde). Sources: UM-BBD_enzymeID:r0338 Relationships: is a type of GO:0016836